{
  "gene": "UniProtKB:Q6W2J9",
  "gene_name": "BCL-6 corepressor",
  "term_label": "transcription corepressor activity",
  "term_id": "GO:0003714",
  "gene_symbol": "BCOR"
}